{
  "gene": "UniProtKB:Q9UII4",
  "term_id": "GO:0061630",
  "term_label": "ubiquitin protein ligase activity",
  "gene_symbol": "HERC5",
  "gene_name": "E3 ISG15--protein ligase HERC5"
}